HULC complex [GO:0033503] (CC) Relationships: is a type of ubiquitin ligase complex [GO:0000151]; is a type of GO:0031371; is part of chromatin [GO:0000785] References: PMID:17363370, PMID:17374714 Sources: GOC:mah Definition: A ubiquitin ligase complex that contains two RING finger proteins, which have ubiquitin ligase activity, in addition to a protein with ubiquitin-conjugating enzyme activity; catalyzes the ubiquitination of histone H2B at lysine 119 (or the equivalent residue). In Schizosaccharomyces the subunits are Rhp6, Shf1, Brl2/Rfp1 and Brl1/Rfp2.